Roundabout signaling pathway involved in axon guidance [GO:2001266] (biological process) Definition: Any Roundabout signaling pathway that is involved in axon guidance. Also known as: ROBO signaling pathway involved in axon guidance, ROBO signaling pathway involved in axon pathfinding, ROBO/SLIT signaling pathway involved in axon guidance, ROBO/SLIT signaling pathway involved in axon pathfinding, Roundabout signaling pathway involved in axon pathfinding, Roundabout signalling pathway involved in axon guidance, Roundabout signalling pathway involved in axon pathfinding, ROBO signaling pathway involved in axon chemotaxis, ROBO signaling pathway involved in axon growth cone guidance, ROBO/SLIT signaling pathway involved in axon chemotaxis, ROBO/SLIT signaling pathway involved in axon growth cone guidance, Roundabout signaling pathway involved in axon chemotaxis, Roundabout signaling pathway involved in axon growth cone guidance, Roundabout signalling pathway involved in axon chemotaxis, Roundabout signalling pathway involved in axon growth cone guidance References: PMID:14527427, PMID:21820427 Sources: GOC:bf Relationships: is a type of GO:0035385; is part of GO:0007411